{
  "term_id": "GO:0051010",
  "term_label": "microtubule plus-end binding",
  "gene_name": "Microtubule-associated protein RP_EB family member 2",
  "gene": "UniProtKB:Q15555",
  "gene_symbol": "MAPRE2"
}